{
  "gene": "UniProtKB:Q7Z7J5",
  "gene_name": "Developmental pluripotency-associated protein 2",
  "term_id": "GO:0048731",
  "gene_symbol": "DPPA2",
  "term_label": "system development"
}